{
  "term_id": "GO:0006915",
  "gene_name": "Caspase-9",
  "gene_symbol": "CASP9",
  "gene": "UniProtKB:P55211",
  "term_label": "apoptotic process"
}